{
  "gene_name": "Four-jointed box protein 1",
  "term_label": "Unknown cellular component",
  "gene_symbol": "FJX1",
  "gene": "UniProtKB:Q86VR8",
  "term_id": "UNKNOWN:0003"
}